{
  "gene_symbol": "FMO4",
  "term_id": "UNKNOWN:0003",
  "gene_name": "Dimethylaniline monooxygenase [N-oxide-forming] 4",
  "term_label": "Unknown cellular component",
  "gene": "UniProtKB:P31512"
}